{
  "term_label": "protein kinase activator activity",
  "gene_name": "Regulator of cell cycle RGCC",
  "gene_symbol": "RGCC",
  "term_id": "GO:0030295",
  "gene": "UniProtKB:Q9H4X1"
}